stearoyl-CoA 9-desaturase activity [GO:0004768] (molecular function) Also known as: acyl-CoA desaturase, delta(9)-desaturase activity, delta9-desaturase, fatty acid desaturase, stearoyl-CoA desaturase activity Relationships: is a type of acyl-CoA desaturase activity [GO:0016215] Definition: Catalysis of the reaction: 2 Fe(II)-[cytochrome b5] + 2 H+ + O2 + octadecanoyl-CoA = (9Z)-octadecenoyl-CoA + 2 Fe(III)-[cytochrome b5] + 2 H2O. Sources: RHEA:19721